{
  "term_id": "GO:0042692",
  "term_label": "muscle cell differentiation",
  "gene_name": "Striated muscle preferentially expressed protein kinase",
  "gene_symbol": "SPEG",
  "gene": "UniProtKB:Q15772"
}